{
  "term_label": "T cell receptor signaling pathway",
  "gene_symbol": "CLEC2B",
  "gene_name": "C-type lectin domain family 2 member B",
  "term_id": "GO:0050852",
  "gene": "UniProtKB:Q92478"
}